{
  "gene_symbol": "TRIM43B",
  "gene": "UniProtKB:A6NCK2",
  "term_id": "GO:0045087",
  "gene_name": "Tripartite motif-containing protein 43B",
  "term_label": "innate immune response"
}